{
  "term_label": "signaling receptor binding",
  "term_id": "GO:0005102",
  "gene_symbol": "ANGPTL6",
  "gene_name": "Angiopoietin-related protein 6",
  "gene": "UniProtKB:Q8NI99"
}